regulation of activated T cell autonomous cell death [GO:0070239] (biological process) Definition: Any process that modulates the occurrence or rate of activated T cell autonomous cell death. Relationships: is a type of regulation of immune system process [GO:0002682]; is a type of regulation of T cell apoptotic process [GO:0070232]; RO_0002211 GO:0070238 Sources: GOC:add, GOC:mtg_apoptosis, ISBN:0781765196 Also known as: regulation of ACAD, regulation of activated T cell apoptosis, regulation of activated cell autonomous cell death, regulation of activated T lymphocyte autonomous cell death, regulation of activated T-cell autonomous cell death, regulation of activated T-lymphocyte autonomous cell death Subtypes: negative regulation of activated T cell autonomous cell death [GO:0070240], positive regulation of activated T cell autonomous cell death [GO:0070241]